{
  "term_id": "GO:0005634",
  "gene": "UniProtKB:Q00534",
  "term_label": "nucleus",
  "gene_name": "Cyclin-dependent kinase 6",
  "gene_symbol": "CDK6"
}